minus-end specific microtubule depolymerization [GO:0036078] (biological process) Definition: The removal of tubulin heterodimers from the minus end of a microtubule. References: PMID:17452528 Sources: GOC:sart Relationships: is a type of microtubule depolymerization [GO:0007019]